{
  "gene_symbol": "CAMK2G",
  "gene": "UniProtKB:Q13555",
  "term_label": "calcium/calmodulin-dependent protein kinase activity",
  "term_id": "GO:0004683",
  "gene_name": "Calcium_calmodulin-dependent protein kinase type II subunit gamma"
}